{
  "term_id": "GO:0045944",
  "gene": "UniProtKB:Q5VV67",
  "term_label": "positive regulation of transcription by RNA polymerase II",
  "gene_symbol": "PPRC1",
  "gene_name": "Peroxisome proliferator-activated receptor gamma coactivator-related protein 1"
}